{
  "gene_name": "Visual system homeobox 2",
  "gene": "UniProtKB:P58304",
  "term_label": "regulation of transcription by RNA polymerase II",
  "gene_symbol": "VSX2",
  "term_id": "GO:0006357"
}